gellan lyase activity [GO:0052762] (molecular function) Definition: Catalysis of the reaction: gellan = n beta-D-4-deoxy-delta4,5-GlcAp-(1->4)-beta-D-Glcp-(1->4)-alpha-L-Rhap-(1->3)-beta-D-Glcp. This reaction is the eliminative cleavage of beta-D-glucopyranosyl-(1->4)-beta-D-glucopyranosyluronate bonds of gellan backbone, releasing tetrasaccharides containing a 4-deoxy-4,5-unsaturated D-glucopyranosyluronic acid at the non-reducing end; in the product, the abbreviations are D-glucose (Glc), D-glucuronic acid (GlcA), and L-rhamnose (Rha). Sources: GOC:mengo_curators, MetaCyc:RXN-12269 Relationships: is a type of GO:0016837